{
  "gene_name": "Calcium homeostasis modulator protein 5",
  "term_label": "plasma membrane",
  "gene": "UniProtKB:Q8N5C1",
  "gene_symbol": "CALHM5",
  "term_id": "GO:0005886"
}